{
  "gene_symbol": "ALKAL2",
  "gene": "UniProtKB:Q6UX46",
  "gene_name": "ALK and LTK ligand 2",
  "term_id": "GO:0030971",
  "term_label": "receptor tyrosine kinase binding"
}